liposaccharide metabolic process [GO:1903509] (biological process) Definition: The chemical reactions and pathways involving liposaccharide. Also known as: liposaccharide metabolism Relationships: is a type of GO:0006629; is_a carbohydrate derivative metabolic process [GO:1901135] References: PMID:9452964 Sources: GOC:TermGenie, GOC:dph, GO_REF:0000068 Subtypes: GO:0006664, GO:0008653